{
  "gene_symbol": "ZNF117",
  "term_id": "GO:0006355",
  "term_label": "regulation of DNA-templated transcription",
  "gene_name": "Zinc finger protein 117",
  "gene": "UniProtKB:Q03924"
}